{
  "term_label": "Unknown molecular function",
  "gene": "UniProtKB:P49755",
  "term_id": "UNKNOWN:0001",
  "gene_name": "Transmembrane emp24 domain-containing protein 10",
  "gene_symbol": "TMED10"
}